{
  "gene": "UniProtKB:P29016",
  "gene_symbol": "CD1B",
  "term_label": "immune response",
  "gene_name": "T-cell surface glycoprotein CD1b",
  "term_id": "GO:0006955"
}